cellular response to flavonoid [GO:1905396] (biological process) Relationships: is a type of cellular response to oxygen-containing compound [GO:1901701]; is a type of response to flavonoid [GO:1905395] References: PMID:22700048 Sources: GOC:TermGenie, GO_REF:0000071 Definition: Any process that results in a change in state or activity of a cell (in terms of movement, secretion, enzyme production, gene expression, etc.) as a result of a flavonoid stimulus. Subtypes: cellular response to catechin [GO:1902169], cellular response to quercetin [GO:1905236]